ureteric bud elongation [GO:0060677] (biological process) References: PMID:16916378 Sources: GOC:dph Relationships: is a type of developmental growth involved in morphogenesis [GO:0060560]; is part of ureteric bud morphogenesis [GO:0060675] Definition: The developmental growth in which the ureteric bud grows along its axis beginning with the growth of the primary ureteric bud and ending when the branches of the bud have elongated.